heme A synthase activity [GO:0120547] (molecular function) Definition: Catalysis of the reaction: Fe(II)-heme o + 2 acceptor + H2O = Fe(II)-heme a + 2 acceptor-H2. The conversion of heme o to heme a occcurs by two successive hydroxylations of the methyl group at C8 using water as the oxygen source. The first hydroxylation forms heme i, the second hydroxylation results in an unstable dihydroxymethyl group, which spontaneously dehydrates, resulting in the formyl group of heme A. References: PMID:30397130 Sources: RHEA:63388 Relationships: is a type of GO:0016725